L-phenylalanine-2-oxoglutarate transaminase activity [GO:0080130] (molecular function) Relationships: is a type of GO:0008793 Also known as: L-phenylalanine:2-oxoglutarate aminotransferase activity, L-phenylalanine:alpha-ketoglutarate aminotransferase activity References: PMID:18394996 Sources: RHEA:25152 Definition: Catalysis of the reaction: L-phenylalanine + 2-oxoglutarate = 3-phenylpyruvate + L-glutamate.